dolichal reductase (NADPH) activity [GO:0160197] (molecular function) Also known as: dolichal reductase [NAD(P)H] activity, dolichal reductase [NAD(P)+] activity References: PMID:38821050 Sources: RHEA:80731 Relationships: is a type of GO:0016628 Definition: Catalysis of the reaction: a di-trans,poly-cis-dolichol + NADP+ = a di-trans,poly-cis-dolichal + NADPH + H+.